{
  "term_label": "plasma membrane",
  "term_id": "GO:0005886",
  "gene": "UniProtKB:P43405",
  "gene_symbol": "SYK",
  "gene_name": "Tyrosine-protein kinase SYK"
}